negative regulation of embryonic skeletal joint development [GO:1902763] (biological process) Also known as: down regulation of embryonic skeletal joint development, down-regulation of embryonic skeletal joint development, downregulation of embryonic skeletal joint development, inhibition of embryonic skeletal joint development References: PMID:16575901 Sources: GOC:TermGenie, GOC:mr, GO_REF:0000058 Definition: Any process that stops, prevents or reduces the frequency, rate or extent of embryonic skeletal joint development. Relationships: is a type of negative regulation of developmental process [GO:0051093]; is a type of GO:1902762; negatively regulates GO:0072498